{
  "term_id": "GO:0006637",
  "term_label": "acyl-CoA metabolic process",
  "gene_name": "Acyl-coenzyme A synthetase ACSM3, mitochondrial",
  "gene_symbol": "ACSM3",
  "gene": "UniProtKB:Q53FZ2"
}